{
  "term_label": "Unknown cellular component",
  "gene_symbol": "CHTF8",
  "gene_name": "Chromosome transmission fidelity protein 8 homolog",
  "gene": "UniProtKB:P0CG13",
  "term_id": "UNKNOWN:0003"
}